{
  "term_id": "UNKNOWN:0001",
  "gene_symbol": "IGLV3-9",
  "gene_name": "Immunoglobulin lambda variable 3-9",
  "term_label": "Unknown molecular function",
  "gene": "UniProtKB:A0A075B6K5"
}